{
  "term_id": "GO:0030424",
  "gene_name": "Vimentin",
  "gene_symbol": "VIM",
  "gene": "UniProtKB:P08670",
  "term_label": "axon"
}